{
  "gene": "UniProtKB:Q9BXS9",
  "gene_name": "Solute carrier family 26 member 6",
  "term_id": "GO:0019531",
  "gene_symbol": "SLC26A6",
  "term_label": "oxalate transmembrane transporter activity"
}